cytoplasmic origin of replication recognition complex [GO:0000809] (cellular component) Definition: A multisubunit complex that is located at the replication origins of a chromosome in the cytoplasm. Sources: GOC:elh Also known as: cytoplasmic ORC, prokaryotic ORC Relationships: is a type of GO:0000808; is part of cytoplasm [GO:0005737]